{
  "gene_name": "Hemoglobin subunit delta",
  "gene_symbol": "HBD",
  "gene": "UniProtKB:P02042",
  "term_id": "GO:0031721",
  "term_label": "hemoglobin alpha binding"
}